{
  "gene": "UniProtKB:Q7Z5P9",
  "term_label": "Unknown molecular function",
  "gene_name": "Mucin-19",
  "gene_symbol": "MUC19",
  "term_id": "UNKNOWN:0001"
}